{
  "term_label": "signaling receptor activity",
  "gene": "UniProtKB:Q9UKX5",
  "term_id": "GO:0038023",
  "gene_name": "Integrin alpha-11",
  "gene_symbol": "ITGA11"
}